{
  "term_label": "RNA polymerase II cis-regulatory region sequence-specific DNA binding",
  "gene": "UniProtKB:O00327",
  "gene_symbol": "BMAL1",
  "term_id": "GO:0000978",
  "gene_name": "Basic helix-loop-helix ARNT-like protein 1"
}